farnesol biosynthetic process [GO:0006715] (biological process) Also known as: farnesol anabolism, farnesol biosynthesis, farnesol formation, farnesol synthesis Sources: ISBN:0198547684 Definition: The chemical reactions and pathways resulting in the formation of the sesquiterpenoid alcohol farnesol, 3,7,11-trimethyl-2,6,10,dodecatrien-1-ol. Relationships: is a type of GO:0016094; is a type of sesquiterpenoid biosynthetic process [GO:0016106]; is a type of farnesol metabolic process [GO:0016487]; is a type of primary alcohol biosynthetic process [GO:0034309]